{
  "gene": "UniProtKB:Q9NQZ3",
  "gene_name": "Deleted in azoospermia protein 1",
  "term_label": "mRNA 3'-UTR binding",
  "term_id": "GO:0003730",
  "gene_symbol": "DAZ1"
}